{
  "term_label": "tissue development",
  "gene_name": "Netrin-4",
  "gene_symbol": "NTN4",
  "term_id": "GO:0009888",
  "gene": "UniProtKB:Q9HB63"
}